{
  "gene": "UniProtKB:Q13432",
  "gene_symbol": "UNC119",
  "gene_name": "Protein unc-119 homolog A",
  "term_label": "spindle pole",
  "term_id": "GO:0000922"
}